{
  "gene_name": "Vesicle transport through interaction with t-SNAREs homolog 1A",
  "term_label": "retrograde transport, endosome to Golgi",
  "gene_symbol": "VTI1A",
  "gene": "UniProtKB:Q96AJ9",
  "term_id": "GO:0042147"
}